{
  "term_label": "transmembrane transporter binding",
  "term_id": "GO:0044325",
  "gene_name": "Ankyrin-1",
  "gene_symbol": "ANK1",
  "gene": "UniProtKB:P16157"
}